{
  "gene_name": "Photoreceptor cilium actin regulator",
  "gene_symbol": "PCARE",
  "term_id": "GO:0001917",
  "gene": "UniProtKB:A6NGG8",
  "term_label": "photoreceptor inner segment"
}